regulation of bioluminescence [GO:1905085] (BP) Relationships: is a type of regulation of metabolic process [GO:0019222]; regulates GO:0008218 Definition: Any process that modulates the frequency, rate or extent of bioluminescence. Subtypes: negative regulation of bioluminescence [GO:1905086], positive regulation of bioluminescence [GO:1905087] References: PMID:10913092 Sources: GOC:BHF, GOC:TermGenie, GOC:rph, GO_REF:0000058